{
  "gene": "UniProtKB:P60900",
  "term_label": "Unknown molecular function",
  "gene_name": "Proteasome subunit alpha type-6",
  "term_id": "UNKNOWN:0001",
  "gene_symbol": "PSMA6"
}